negative regulation of lipid metabolic process [GO:0045833] (biological process) Definition: Any process that stops, prevents, or reduces the frequency, rate or extent of the chemical reactions and pathways involving lipids. Sources: GOC:go_curators Also known as: down regulation of lipid metabolic process, down-regulation of lipid metabolic process, downregulation of lipid metabolic process, negative regulation of lipid metabolism, inhibition of lipid metabolic process Relationships: is a type of negative regulation of metabolic process [GO:0009892]; is a type of regulation of lipid metabolic process [GO:0019216]; negatively regulates GO:0006629 Subtypes: negative regulation of isoprenoid metabolic process [GO:0045827], negative regulation of fatty acid metabolic process [GO:0045922], negative regulation of steroid metabolic process [GO:0045939], negative regulation of lipid catabolic process [GO:0050995], negative regulation of lipid biosynthetic process [GO:0051055], negative regulation of lipoprotein lipid oxidation [GO:0060588], negative regulation of triglyceride metabolic process [GO:0090209], negative regulation of phospholipid metabolic process [GO:1903726]